glycyl-tRNA aminoacylation [GO:0006426] (biological process) Subtypes: mitochondrial glycyl-tRNA aminoacylation [GO:0070150] Relationships: is a type of tRNA aminoacylation for protein translation [GO:0006418] Sources: GOC:mcc, ISBN:0716730510 Definition: The process of coupling glycine to glycyl-tRNA, catalyzed by glycyl-tRNA synthetase. The glycyll-tRNA synthetase is a class-II synthetase. The activated amino acid is transferred to the 3'-OH group of a glycine-accepting tRNA.